{
  "term_id": "UNKNOWN:0001",
  "gene_name": "Protein virilizer homolog",
  "gene": "UniProtKB:Q69YN4",
  "gene_symbol": "VIRMA",
  "term_label": "Unknown molecular function"
}